hemoglobin beta binding [GO:0031722] (molecular function) Sources: GOC:mah Definition: Binding to a hemoglobin beta chain. Relationships: is a type of GO:0030492